{
  "gene_name": "Fatty acyl-CoA reductase 2",
  "term_label": "peroxisome",
  "gene_symbol": "FAR2",
  "gene": "UniProtKB:Q96K12",
  "term_id": "GO:0005777"
}